{
  "gene_symbol": "CAPN11",
  "term_label": "cytoplasm",
  "gene_name": "Calpain-11",
  "term_id": "GO:0005737",
  "gene": "UniProtKB:Q9UMQ6"
}